auxin:proton symporter activity [GO:0009672] (molecular function) References: PMID:8688077 Definition: Enables the transfer of a solute or solutes from one side of a membrane to the other according to the reaction: auxin(out) + H+(out) = auxin(in) + H+(in). Also known as: auxin:hydrogen symporter activity Relationships: is a type of solute:proton symporter activity [GO:0015295]; is a type of GO:0080161